{
  "gene_symbol": "PRB3",
  "term_label": "Unknown biological process",
  "gene_name": "Basic salivary proline-rich protein 3",
  "gene": "UniProtKB:Q04118",
  "term_id": "UNKNOWN:0002"
}